ubiquitin ligase complex scaffold activity [GO:0160072] (molecular function) Relationships: is_a protein-macromolecule adaptor activity [GO:0030674] Also known as: core protein activity for the CUL-RING ubiquitin ligase complex, core protein activity for the Cullin-RING ubiquitin ligase complex References: PMID:27664236 Definition: The binding activity of a molecule that brings together an ubiquitin ligase and an ubiquitin ligase-substrate adaptor, permitting those molecules to function in a coordinated way.